intermediate filament polymerization [GO:0045107] (biological process) Definition: Assembly of intermediate filaments by the addition of component monomers to a filament. Polymerization of intermediate filament proteins results from interactions among several distinct binding sites on the constituent proteins. Nuclear lamin head-to-tail polymers arise from one such interaction. Deletion analysis localized the binding sites to the ends of the rod domain that are highly conserved among all intermediate filament proteins. Data indicate that one type of interaction in intermediate filament protein polymerization is the longitudinal binding of dimers via the conserved end segments of the coiled-coil rod domain. Relationships: is_a intermediate filament polymerization or depolymerization [GO:0045105]; is a type of protein polymerization [GO:0051258] Regulation: regulated by regulation of intermediate filament polymerization [GO:0030839]; negatively regulated by negative regulation of intermediate filament polymerization [GO:0030840]; positively regulated by GO:0030841 References: PMID:8776884 Sources: GOC:mah